{
  "term_label": "glucose metabolic process",
  "gene_symbol": "HKDC1",
  "gene": "UniProtKB:Q2TB90",
  "gene_name": "Hexokinase HKDC1",
  "term_id": "GO:0006006"
}